telomere organization [GO:0032200] (biological process) Relationships: is a type of GO:0051276 Definition: A process that is carried out at the cellular level which results in the assembly, arrangement of constituent parts, or disassembly of telomeres, terminal regions of a linear chromosome that include the telomeric DNA repeats and associated proteins. Also known as: chromosome organization, telomeric, organization of chromosome, telomeric region, telomere organisation, telomere organization and biogenesis Subtypes: telomere maintenance [GO:0000723], telomere assembly [GO:0032202] Sources: GOC:dph, GOC:jl, GOC:mah